{
  "gene": "UniProtKB:O60858",
  "term_id": "GO:0016239",
  "term_label": "positive regulation of macroautophagy",
  "gene_symbol": "TRIM13",
  "gene_name": "E3 ubiquitin-protein ligase TRIM13"
}